pyrimidine nucleoside metabolic process [GO:0006213] (biological process) Sources: GOC:jl, ISBN:0140512713 Relationships: is a type of nucleoside metabolic process [GO:0009116]; is a type of pyrimidine-containing compound metabolic process [GO:0072527] Also known as: pyrimidine metabolic process, pyrimidine metabolism, pyrimidine nucleoside metabolism Subtypes: pyrimidine nucleoside interconversion [GO:0019689], GO:0046125, GO:0046131, GO:0046134, pyrimidine nucleoside catabolic process [GO:0046135] Definition: The chemical reactions and pathways involving any pyrimidine nucleoside, one of a family of organic molecules consisting of a pyrimidine base covalently bonded to ribose (a ribonucleoside) or deoxyribose (a deoxyribonucleoside).